{
  "gene_symbol": "AKT1S1",
  "gene": "UniProtKB:Q96B36",
  "term_id": "GO:1904262",
  "term_label": "negative regulation of TORC1 signaling",
  "gene_name": "Proline-rich AKT1 substrate 1"
}